{
  "term_label": "clathrin coat of coated pit",
  "term_id": "GO:0030132",
  "gene_symbol": "EPS15L1",
  "gene_name": "Epidermal growth factor receptor substrate 15-like 1",
  "gene": "UniProtKB:Q9UBC2"
}